superoxide dismutase complex [GO:1902693] (cellular component) References: PMID:10026301 Sources: GOC:TermGenie, GOC:bhm, GO_REF:0000088 Definition: A protein complex which is capable of superoxide dismutase activity. Relationships: is a type of GO:1990204 Note: An example of this is SOD1 in Saccharomyces cerevisiae S288c (UniProt symbol P00445) in PMID:10026301.